L-arginine biosynthetic process via ornithine [GO:0042450] (biological process) Also known as: arginine anabolism via ornithine, arginine biosynthesis, acetylated pathway, arginine formation via ornithine, arginine synthesis via ornithine, classical arginine biosynthesis pathway Definition: The chemical reactions and pathways resulting in the formation of arginine (2-amino-5-guanidinopentanoic acid) via the intermediate compound ornithine. Regulation: regulated by regulation of arginine biosynthetic process via ornithine [GO:2000013] Relationships: is a type of L-arginine biosynthetic process [GO:0006526] Sources: GOC:jl